{
  "gene_symbol": "ZDHHC5",
  "gene": "UniProtKB:Q9C0B5",
  "gene_name": "Palmitoyltransferase ZDHHC5",
  "term_id": "GO:0016409",
  "term_label": "palmitoyltransferase activity"
}